{
  "gene_symbol": "OR11A1",
  "gene_name": "Olfactory receptor 11A1",
  "gene": "UniProtKB:Q9GZK7",
  "term_id": "UNKNOWN:0003",
  "term_label": "Unknown cellular component"
}